thermomorphogenesis [GO:0140919] (biological process) Relationships: is a type of response to temperature stimulus [GO:0009266]; is a type of GO:0009791 References: PMID:27250752 Regulation: regulated by GO:0140920; negatively regulated by negative regulation of thermomorphogenesis [GO:0140921]; positively regulated by positive regulation of thermomorphogenesis [GO:0140922] Definition: The suite of morphological and architectural changes in an organism induced by high ambient temperatures, below the heat-stress range.